single base insertion or deletion binding [GO:0032138] (molecular function) Subtypes: GO:0032140, single cytosine insertion binding [GO:0032141], single guanine insertion binding [GO:0032142], single thymine insertion binding [GO:0032143] Definition: Binding to a double-stranded DNA region containing a single base insertion or deletion. Also known as: single base insertion binding Sources: GOC:vk Relationships: is_a GO:0032135